{
  "term_label": "Unknown molecular function",
  "gene_symbol": "DSCC1",
  "gene": "UniProtKB:Q9BVC3",
  "term_id": "UNKNOWN:0001",
  "gene_name": "Sister chromatid cohesion protein DCC1"
}